{
  "term_label": "adenyl-nucleotide exchange factor activity",
  "gene_symbol": "BAG1",
  "gene_name": "BAG family molecular chaperone regulator 1",
  "term_id": "GO:0000774",
  "gene": "UniProtKB:Q99933"
}